{
  "term_label": "Unknown molecular function",
  "gene": "UniProtKB:A6NKL6",
  "term_id": "UNKNOWN:0001",
  "gene_name": "Transmembrane protein 200C",
  "gene_symbol": "TMEM200C"
}